{
  "gene": "UniProtKB:Q08050",
  "term_label": "RNA polymerase II transcription regulatory region sequence-specific DNA binding",
  "term_id": "GO:0000977",
  "gene_name": "Forkhead box protein M1",
  "gene_symbol": "FOXM1"
}